{
  "gene_name": "Pogo transposable element with KRAB domain",
  "term_label": "nucleus",
  "term_id": "GO:0005634",
  "gene": "UniProtKB:Q9P215",
  "gene_symbol": "POGK"
}